{
  "term_id": "GO:0005737",
  "gene": "UniProtKB:Q9H2C0",
  "term_label": "cytoplasm",
  "gene_symbol": "GAN",
  "gene_name": "Gigaxonin"
}